alpha-ketoester reductase (NADPH) activity [GO:0051269] (MF) References: PMID:15564669 Sources: RHEA:80767 Definition: Catalysis of the reaction: alpha-ketoester + H+ + NADPH = (R)-hydroxy ester + NADP+. Relationships: is a type of oxidoreductase activity, acting on the aldehyde or oxo group of donors, NAD or NADP as acceptor [GO:0016620]